adenosine metabolic process [GO:0046085] (biological process) Relationships: is a type of purine ribonucleoside metabolic process [GO:0046128] Also known as: adenosine metabolism Sources: GOC:go_curators Subtypes: adenosine catabolic process [GO:0006154], adenosine biosynthetic process [GO:0046086] Definition: The chemical reactions and pathways involving adenosine, adenine riboside, a ribonucleoside found widely distributed in cells of every type as the free nucleoside and in combination in nucleic acids and various nucleoside coenzymes.